anti-Mullerian hormone receptor activity [GO:1990272] (molecular function) Note: An example of this is Amdh2 in M. musculus, UniprotKB:Q8K592-1 in PMID:23624077. Relationships: is a type of protein-hormone receptor activity [GO:0016500]; is part of anti-Mullerian hormone receptor signaling pathway [GO:1990262] Definition: Combining with anti-Mullerian hormone to initiate a change in cell activity. References: PMID:23624077 Sources: GOC:hjd